{
  "term_label": "negative regulation of cell population proliferation",
  "gene_name": "Wilms tumor protein",
  "gene_symbol": "WT1",
  "term_id": "GO:0008285",
  "gene": "UniProtKB:P19544"
}